{
  "gene_name": "Immunoglobulin heavy variable 3-20",
  "gene_symbol": "IGHV3-20",
  "term_label": "immunoglobulin mediated immune response",
  "gene": "UniProtKB:A0A0C4DH32",
  "term_id": "GO:0016064"
}